{
  "gene_name": "Keratin-associated protein 5-5",
  "term_id": "UNKNOWN:0003",
  "term_label": "Unknown cellular component",
  "gene_symbol": "KRTAP5-5",
  "gene": "UniProtKB:Q701N2"
}